{
  "gene": "UniProtKB:Q8NAM6",
  "term_id": "GO:0000978",
  "term_label": "RNA polymerase II cis-regulatory region sequence-specific DNA binding",
  "gene_name": "Zinc finger and SCAN domain-containing protein 4",
  "gene_symbol": "ZSCAN4"
}